{
  "gene": "UniProtKB:P54252",
  "term_id": "GO:1904262",
  "gene_name": "Ataxin-3",
  "gene_symbol": "ATXN3",
  "term_label": "negative regulation of TORC1 signaling"
}